{
  "gene_name": "Potassium_sodium hyperpolarization-activated cyclic nucleotide-gated channel 3",
  "term_id": "GO:0098855",
  "gene_symbol": "HCN3",
  "term_label": "HCN channel complex",
  "gene": "UniProtKB:Q9P1Z3"
}